neuron projection morphogenesis [GO:0048812] (biological process) Definition: The process in which the anatomical structures of a neuron projection are generated and organized. A neuron projection is any process extending from a neural cell, such as axons or dendrites. Sources: GOC:mah Also known as: neurite biosynthesis, neurite formation, neurite growth, neurite morphogenesis Relationships: is a type of plasma membrane bounded cell projection morphogenesis [GO:0120039]; is part of neuron projection development [GO:0031175] Subtypes: axonogenesis [GO:0007409], dendrite morphogenesis [GO:0048813], dendritic spine morphogenesis [GO:0060997], rhabdomere morphogenesis [GO:0061541], GO:0140058